glucose catabolic process to lactate via pyruvate [GO:0019661] (biological process) Regulation: regulated by regulation of glucose catabolic process to lactate via pyruvate [GO:1904023]; negatively regulated by negative regulation of glucose catabolic process to lactate via pyruvate [GO:1904024]; positively regulated by positive regulation of glucose catabolic process to lactate via pyruvate [GO:1904025] Sources: GOC:jl Also known as: glucose fermentation to lactate via pyruvate, homofermentation, homofermentative lactate fermentation, homofermentative pathway, homolactate fermentation, homolactic fermentation Relationships: is a type of glucose catabolic process to lactate [GO:0019659]; has part L(+)-lactate biosynthetic process from pyruvate [GO:0019246]; has part GO:0061621 Definition: The anaerobic enzymatic chemical reactions and pathways resulting in the breakdown of glucose to lactate, via canonical glycolysis, yielding energy in the form of adenosine triphosphate (ATP).